{
  "gene_symbol": "RET",
  "gene_name": "Proto-oncogene tyrosine-protein kinase receptor Ret",
  "term_label": "transmembrane receptor protein tyrosine kinase activity",
  "gene": "UniProtKB:P07949",
  "term_id": "GO:0004714"
}